{
  "gene_name": "Chymotrypsin-like elastase family member 2A",
  "gene_symbol": "CELA2A",
  "term_id": "GO:0004252",
  "term_label": "serine-type endopeptidase activity",
  "gene": "UniProtKB:P08217"
}